{
  "gene": "UniProtKB:P31213",
  "term_label": "neuronal cell body",
  "term_id": "GO:0043025",
  "gene_name": "3-oxo-5-alpha-steroid 4-dehydrogenase 2",
  "gene_symbol": "SRD5A2"
}